{
  "term_label": "Unknown biological process",
  "gene_name": "Putative uncharacterized protein encoded by MIR22HG",
  "term_id": "UNKNOWN:0002",
  "gene": "UniProtKB:Q0VDD5",
  "gene_symbol": "MIR22HG"
}